{
  "gene_symbol": "KREMEN2",
  "gene_name": "Kremen protein 2",
  "term_label": "transmembrane signaling receptor activity",
  "term_id": "GO:0004888",
  "gene": "UniProtKB:Q8NCW0"
}